cellular response to tumor cell [GO:0071228] (biological process) Relationships: is a type of response to tumor cell [GO:0002347]; is a type of cellular response to biotic stimulus [GO:0071216] Sources: GOC:mah Definition: Any process that results in a change in state or activity of a cell (in terms of movement, secretion, enzyme production, gene expression, etc.) as a result of a stimulus from a tumor cell.